{
  "gene": "UniProtKB:Q9UPN6",
  "gene_symbol": "SCAF8",
  "gene_name": "SR-related and CTD-associated factor 8",
  "term_label": "RNA polymerase II complex binding",
  "term_id": "GO:0000993"
}